nitrogen cycle metabolic process [GO:0071941] (biological process) Subtypes: nitrogen fixation [GO:0009399], anaerobic respiration, using ammonium as electron donor [GO:0019331], denitrification pathway [GO:0019333], aerobic respiration, using ammonia as electron donor [GO:0019409], urea metabolic process [GO:0019627], nitrate assimilation [GO:0042128] References: PMID:16675690 Sources: GOC:mah, Wikipedia:Nitrogen_cycle Relationships: is_a GO:0008152 Regulation: regulated by regulation of nitrogen cycle metabolic process [GO:1903314]; negatively regulated by GO:1903315; positively regulated by positive regulation of nitrogen cycle metabolic process [GO:1903316] Definition: A nitrogen compound metabolic process that contributes to the nitrogen cycle. The nitrogen cycle is a series of metabolic pathways by which nitrogen is converted between various forms and redox states; it encompasses pathways in which nitrogen is acted upon directly, such as nitrification, denitrification, nitrogen fixation, and mineralization.